{
  "gene": "UniProtKB:P17482",
  "term_label": "RNA polymerase II cis-regulatory region sequence-specific DNA binding",
  "term_id": "GO:0000978",
  "gene_name": "Homeobox protein Hox-B9",
  "gene_symbol": "HOXB9"
}